viral DNA genome packaging, headful [GO:0098006] (biological process) Definition: The encapsulation of the viral genome within the capsid where DNA is packaged into the capsid until the capsid is full. Sources: GOC:bm Also known as: phage headful packaging Note: Generalized transducing phages usually use this mode of DNA packaging. Relationships: is a type of viral DNA genome packaging [GO:0019073]